histone chaperone activity [GO:0140713] (molecular function) Definition: Binding to and carrying a histone or a histone complex to unload or deposit it as a nucleosome. The histone can be newly synthesized or result from nucleosome disassembly (either spontaneously, or by a histone chaperone). Subtypes: H3-H4 histone complex chaperone activity [GO:0000510], GO:0000511, ATP-dependent histone chaperone activity [GO:0140674], H1 histone chaperone activity [GO:0140890] Also known as: histone carrier activity, nucleosome remodeling activity References: PMID:26459557 Relationships: is_a GO:0140597; has part histone binding [GO:0042393]